chitin-based cuticle sclerotization by protein cross-linking [GO:0036341] (BP) Also known as: chitin-based cuticle sclerotization by protein cross-linking and cuticle tanning Relationships: is a type of chitin-based cuticle sclerotization [GO:0007593] Definition: The process of hardening of a chitin-based cuticle by protein cross-linking, and the incorporation of phenolic precursors. This mechanism of cuticle hardening occurs in insects and is usually accompanied by darkening of the cuticle. Sources: GOC:bf, GOC:sart